{
  "gene_name": "StAR-related lipid transfer protein 4",
  "term_label": "endoplasmic reticulum",
  "gene": "UniProtKB:Q96DR4",
  "gene_symbol": "STARD4",
  "term_id": "GO:0005783"
}